{
  "term_label": "DNA polymerase binding",
  "gene_symbol": "CDT1",
  "term_id": "GO:0070182",
  "gene_name": "DNA replication factor Cdt1",
  "gene": "UniProtKB:Q9H211"
}